{
  "term_label": "mitochondrial large ribosomal subunit",
  "term_id": "GO:0005762",
  "gene": "UniProtKB:P49406",
  "gene_symbol": "MRPL19",
  "gene_name": "Large ribosomal subunit protein bL19m"
}